{
  "gene_name": "Putative PIN1-like protein",
  "gene_symbol": "PIN1P1",
  "gene": "UniProtKB:O15428",
  "term_id": "UNKNOWN:0002",
  "term_label": "Unknown biological process"
}